mitogen-activated protein kinase kinase kinase kinase binding [GO:0033161] (molecular function) Also known as: MAPKKKK binding Sources: GOC:mah Definition: Binding to a mitogen-activated protein kinase kinase kinase kinase, a protein that can phosphorylate a MAP kinase kinase kinase. Relationships: is a type of GO:0019901